{
  "gene_symbol": "GGCX",
  "gene_name": "Vitamin K-dependent gamma-carboxylase",
  "gene": "UniProtKB:P38435",
  "term_id": "GO:0042373",
  "term_label": "vitamin K metabolic process"
}